{
  "gene": "UniProtKB:O00160",
  "gene_name": "Unconventional myosin-If",
  "gene_symbol": "MYO1F",
  "term_label": "microvillus",
  "term_id": "GO:0005902"
}